{
  "term_id": "GO:1902035",
  "gene_name": "Thrombopoietin",
  "gene": "UniProtKB:P40225",
  "term_label": "positive regulation of hematopoietic stem cell proliferation",
  "gene_symbol": "THPO"
}